D-galactose-1-phosphate phosphatase activity [GO:0070457] (molecular function) Relationships: is a type of galactose-1-phosphate phosphatase activity [GO:0070456] Definition: Catalysis of the reaction: D-galactose-1-phosphate + H2O = D-galactose + phosphate. References: PMID:9462881 Sources: GOC:mah